{
  "term_id": "GO:1905394",
  "term_label": "retromer complex binding",
  "gene_symbol": "M6PR",
  "gene_name": "Cation-dependent mannose-6-phosphate receptor",
  "gene": "UniProtKB:P20645"
}